{
  "gene_name": "Ras-related protein Rab-7a",
  "term_label": "endosome to lysosome transport",
  "gene_symbol": "RAB7A",
  "term_id": "GO:0008333",
  "gene": "UniProtKB:P51149"
}